{
  "gene": "UniProtKB:A6NJZ3",
  "term_id": "GO:0004984",
  "gene_symbol": "OR6C65",
  "term_label": "olfactory receptor activity",
  "gene_name": "Olfactory receptor 6C65"
}